regulation of T cell activation [GO:0050863] (biological process) Also known as: regulation of T lymphocyte activation, regulation of T-cell activation, regulation of T-lymphocyte activation Relationships: is a type of GO:0051249; regulates T cell activation [GO:0042110] Sources: GOC:ai Subtypes: regulation of T cell proliferation [GO:0042129], regulation of T cell differentiation [GO:0045580], GO:0046634, regulation of gamma-delta T cell activation [GO:0046643], negative regulation of T cell activation [GO:0050868], positive regulation of T cell activation [GO:0050870], GO:2000523, GO:2000567, regulation of T cell activation via T cell receptor contact with antigen bound to MHC molecule on antigen presenting cell [GO:2001188] Definition: Any process that modulates the frequency, rate or extent of T cell activation.